{
  "term_label": "inflammatory response",
  "term_id": "GO:0006954",
  "gene_name": "C-C motif chemokine 3",
  "gene_symbol": "CCL3",
  "gene": "UniProtKB:P10147"
}